{
  "gene": "UniProtKB:Q86V42",
  "term_id": "UNKNOWN:0003",
  "gene_name": "Protein FAM124A",
  "term_label": "Unknown cellular component",
  "gene_symbol": "FAM124A"
}